{
  "gene": "UniProtKB:Q8N349",
  "term_id": "GO:0004984",
  "gene_symbol": "OR2L13",
  "term_label": "olfactory receptor activity",
  "gene_name": "Olfactory receptor 2L13"
}